{
  "gene_name": "Metallothionein-1F",
  "gene": "UniProtKB:P04733",
  "term_label": "cellular response to copper ion",
  "gene_symbol": "MT1F",
  "term_id": "GO:0071280"
}